{
  "gene_name": "Frizzled-1",
  "term_label": "canonical Wnt signaling pathway",
  "gene_symbol": "FZD1",
  "term_id": "GO:0060070",
  "gene": "UniProtKB:Q9UP38"
}